regulation of fat cell proliferation [GO:0070344] (biological process) Also known as: regulation of adipocyte proliferation, regulation of adipose cell proliferation Subtypes: negative regulation of fat cell proliferation [GO:0070345], positive regulation of fat cell proliferation [GO:0070346], regulation of brown fat cell proliferation [GO:0070347], regulation of white fat cell proliferation [GO:0070350] Relationships: is a type of regulation of cell population proliferation [GO:0042127]; regulates fat cell proliferation [GO:0070341] Sources: GOC:mah, GOC:sl Definition: Any process that modulates the frequency, rate or extent of fat cell proliferation.